maintenance of DNA repeat elements [GO:0043570] (biological process) Definition: Any process involved in sustaining the fidelity and copy number of DNA repeat elements. Sources: GOC:jl Relationships: is a type of DNA metabolic process [GO:0006259]; is a type of chromosome organization [GO:0051276] Subtypes: maintenance of DNA trinucleotide repeats [GO:0035753], maintenance of rDNA [GO:0043007], maintenance of CRISPR repeat elements [GO:0043571]